{
  "term_label": "Unknown cellular component",
  "gene_symbol": "ZNF576",
  "gene_name": "Zinc finger protein 576",
  "term_id": "UNKNOWN:0003",
  "gene": "UniProtKB:Q9H609"
}